NAD-dependent protein lysine deacylase activity [GO:0141218] (molecular function) Also known as: protein lysine deacylase activity Relationships: is a type of acyltransferase activity, transferring groups other than amino-acyl groups [GO:0016747]; is a type of catalytic activity, acting on a protein [GO:0140096]; is a type of deacylase activity [GO:0160215] Subtypes: NAD-dependent protein lysine deacetylase activity [GO:0034979], protein-succinyllysine desuccinylase activity [GO:0036055], protein-glutaryllysine deglutarylase activity [GO:0061697], GO:0106231 Definition: Catalysis of the reaction: N6-acyl-L-lysyl-[protein] + NAD+ + H2O = 2''-O-acyl-ADP-D-ribose + nicotinamide + L-lysyl-[protein]. References: PMID:35044827 Sources: RHEA:54172